nematode pharyngeal muscle development [GO:0160096] (biological process) Relationships: is a type of muscle organ development [GO:0007517]; is part of nematode pharynx development [GO:0160094] Definition: The process whose specific outcome is the progression of the nematode pharyngeal muscle over time, from its formation to the mature structure. Sources: GOC:go_curators